histone H4R3 arginine deiminase activity [GO:0140809] (molecular function) Note: Note that the residue position corresponds to the canonical human H4 histone (UniProtKB:P02309); this residue is conserved across all eukaryotes. Note that the initiation methionine is cleaved, so the first residue is S1. The substrate for histone deiminase may be methyl-arginine, rather than arginine (see PMID:35197210 and PMID:16567635). Definition: Catalysis of the reaction: H2O + histone H4 L-arginyl (position 3)= histone H4 L-citrullyl (position 3) + NH4+, resulting in histone H4 citrullination at position 3. Relationships: is a type of GO:0140794 Also known as: H4-R3 citrullination, histone H4-R3 arginine deiminase activity, histone-arginine deiminase activity (H4-R3 specific) References: PMID:16567635